{
  "term_id": "GO:0015267",
  "term_label": "channel activity",
  "gene": "UniProtKB:Q16548",
  "gene_symbol": "BCL2A1",
  "gene_name": "Bcl-2-related protein A1"
}